protein tyrosine/threonine phosphatase activity [GO:0008330] (molecular function) Definition: Catalysis of the reactions: protein threonine phosphate + H2O = protein threonine + phosphate; and protein tyrosine phosphate + H2O = protein tyrosine + phosphate. Sources: GOC:mah Relationships: is a type of GO:0004721